{
  "gene_name": "Taste receptor type 2 member 45",
  "gene": "UniProtKB:P59539",
  "term_id": "GO:0016020",
  "term_label": "membrane",
  "gene_symbol": "TAS2R45"
}